{
  "gene_symbol": "YTHDC2",
  "gene": "UniProtKB:Q9H6S0",
  "term_id": "GO:0003723",
  "gene_name": "3'-5' RNA helicase YTHDC2",
  "term_label": "RNA binding"
}